ornithine carbamoyltransferase inhibitor complex [GO:1903269] (cellular component) Also known as: OTC-ARGI complex, ornithine carbamoyltransferase arginase complex Note: An example of this is ARGI in Saccharomyces cerevisiae (P00812) in PMID:12679340 (inferred from direct assay). Definition: A protein complex which is capable of ornithine carbamoyltransferase inhibitor activity. Relationships: is a type of catalytic complex [GO:1902494] References: PMID:12679340 Sources: GOC:TermGenie, GOC:bhm, GO_REF:0000088